{
  "gene_name": "Nuclear pore complex-interacting protein family member B9",
  "gene": "UniProtKB:F8W1W9",
  "gene_symbol": "NPIPB9",
  "term_id": "UNKNOWN:0002",
  "term_label": "Unknown biological process"
}